{
  "gene_name": "Transmembrane protein 106C",
  "gene": "UniProtKB:Q9BVX2",
  "term_label": "Unknown biological process",
  "term_id": "UNKNOWN:0002",
  "gene_symbol": "TMEM106C"
}